purine nucleoside bisphosphate biosynthetic process [GO:0034033] (biological process) Definition: The chemical reactions and pathways resulting in the formation of a purine nucleoside bisphosphate, a compound consisting of a purine base linked to a deoxyribose or ribose sugar esterified with one phosphate group attached to each of two different hydroxyl groups on the sugar. Subtypes: purine ribonucleoside bisphosphate biosynthetic process [GO:0034036] Relationships: is a type of nucleoside bisphosphate biosynthetic process [GO:0033866]; is a type of GO:0034032; is a type of purine-containing compound biosynthetic process [GO:0072522] Also known as: purine nucleoside bisphosphate anabolism, purine nucleoside bisphosphate biosynthesis, purine nucleoside bisphosphate formation, purine nucleoside bisphosphate synthesis Sources: GOC:mah, GOC:pde